{
  "gene_name": "Rho GTPase-activating protein 26",
  "gene_symbol": "ARHGAP26",
  "gene": "UniProtKB:Q9UNA1",
  "term_id": "GO:0005096",
  "term_label": "GTPase activator activity"
}